{
  "gene_name": "Cytochrome P450 4Z1",
  "term_id": "UNKNOWN:0002",
  "term_label": "Unknown biological process",
  "gene": "UniProtKB:Q86W10",
  "gene_symbol": "CYP4Z1"
}